{
  "gene": "UniProtKB:Q93034",
  "term_id": "GO:0005634",
  "term_label": "nucleus",
  "gene_symbol": "CUL5",
  "gene_name": "Cullin-5"
}